{
  "gene": "UniProtKB:Q9NRC9",
  "term_id": "UNKNOWN:0003",
  "gene_name": "Otoraplin",
  "gene_symbol": "OTOR",
  "term_label": "Unknown cellular component"
}